{
  "gene": "UniProtKB:Q96S65",
  "gene_name": "Cysteine_serine-rich nuclear protein 1",
  "term_label": "sequence-specific DNA binding",
  "gene_symbol": "CSRNP1",
  "term_id": "GO:0043565"
}